{
  "term_id": "UNKNOWN:0001",
  "gene_name": "Putative UPF0607 protein ENSP00000383783",
  "gene_symbol": "A8MUI8",
  "term_label": "Unknown molecular function",
  "gene": "UniProtKB:A8MUI8"
}